{
  "gene_name": "Mid1-interacting protein 1",
  "term_id": "GO:0046890",
  "gene": "UniProtKB:Q9NPA3",
  "term_label": "regulation of lipid biosynthetic process",
  "gene_symbol": "MID1IP1"
}